viroplasm viral factory [GO:0039716] (cellular component) Relationships: is a type of cytoplasmic viral factory [GO:0039714] Definition: A cytoplasmic viral factory that is electron dense due to high levels of viral RNA. Produced by nucleo-cytoplasmic large DNA viruses (NCLDV) like Poxviridae, Asfarviridae and Iridoviridae, and dsRNA viruses like Reoviridae. Sources: VZ:1951, Wikipedia:Viroplasm